{
  "term_id": "GO:0006979",
  "gene_symbol": "OXR1",
  "gene_name": "Oxidation resistance protein 1",
  "term_label": "response to oxidative stress",
  "gene": "UniProtKB:Q8N573"
}